{
  "gene_name": "Cyclin-G2",
  "term_id": "GO:0016538",
  "gene_symbol": "CCNG2",
  "gene": "UniProtKB:Q16589",
  "term_label": "cyclin-dependent protein serine/threonine kinase regulator activity"
}